{
  "term_id": "GO:0030134",
  "gene_symbol": "KLHL12",
  "term_label": "COPII-coated ER to Golgi transport vesicle",
  "gene": "UniProtKB:Q53G59",
  "gene_name": "Kelch-like protein 12"
}